regulation of vasoconstriction by circulating norepinephrine [GO:0003117] (biological process) Definition: Any process that modulates the frequency, rate or extent of reductions in the diameter of blood vessels as a result of secretion of norepinephrine into the bloodstream. Sources: GOC:mtg_cardio Also known as: regulation of vasoconstriction by circulating noradrenaline Relationships: is a type of GO:0003116